male germline ring canal formation [GO:0030726] (biological process) Also known as: spermatocyte ring canal formation, testicular ring canal formation Sources: ISBN:0879694238 Definition: Formation of the intercellular bridges that connect the germ-line cells of a male cyst. Relationships: is a type of germline ring canal formation [GO:0030725]; is part of spermatogenesis [GO:0007283]